{
  "term_id": "UNKNOWN:0002",
  "gene": "UniProtKB:A6NNY8",
  "gene_name": "Ubiquitin carboxyl-terminal hydrolase 27",
  "term_label": "Unknown biological process",
  "gene_symbol": "USP27X"
}